{
  "gene": "UniProtKB:P16150",
  "term_label": "regulation of immune response",
  "term_id": "GO:0050776",
  "gene_name": "Leukosialin",
  "gene_symbol": "SPN"
}